{
  "term_label": "store-operated calcium entry",
  "gene": "UniProtKB:Q86TD4",
  "gene_symbol": "SRL",
  "term_id": "GO:0002115",
  "gene_name": "Sarcalumenin"
}